protein complex oligomerization [GO:0051259] (biological process) Definition: The process of creating protein oligomers, compounds composed of a small number, usually between three and ten, of component monomers; protein oligomers may be composed of different or identical monomers. Oligomers may be formed by the polymerization of a number of monomers or the depolymerization of a large protein polymer. Regulation: regulated by regulation of protein oligomerization [GO:0032459]; negatively regulated by negative regulation of protein oligomerization [GO:0032460]; positively regulated by GO:0032461 Also known as: protein oligomer biosynthesis, protein oligomer biosynthetic process, protein oligomer assembly, protein oligomer formation, protein oligomerization, protein multimerization References: PMID:18293929 Sources: GOC:ai Subtypes: protein hexamerization [GO:0034214], protein homooligomerization [GO:0051260], protein tetramerization [GO:0051262], protein heterooligomerization [GO:0051291], protein trimerization [GO:0070206] Relationships: is a type of protein-containing complex assembly [GO:0065003]